{
  "term_label": "Unknown cellular component",
  "gene_name": "Putative coiled-coil domain-containing protein 144 N-terminal-like",
  "gene": "UniProtKB:Q6NUI1",
  "gene_symbol": "CCDC144NL",
  "term_id": "UNKNOWN:0003"
}